{
  "term_id": "GO:0031012",
  "term_label": "extracellular matrix",
  "gene": "UniProtKB:Q96RW7",
  "gene_name": "Hemicentin-1",
  "gene_symbol": "HMCN1"
}